{
  "term_label": "cytoplasm",
  "gene": "UniProtKB:O76054",
  "gene_symbol": "SEC14L2",
  "gene_name": "SEC14-like protein 2",
  "term_id": "GO:0005737"
}